{
  "gene_symbol": "TNRC6B",
  "term_label": "miRNA-mediated post-transcriptional gene silencing",
  "gene": "UniProtKB:Q9UPQ9",
  "gene_name": "Trinucleotide repeat-containing gene 6B protein",
  "term_id": "GO:0035195"
}